{
  "term_id": "GO:0050901",
  "term_label": "leukocyte tethering or rolling",
  "gene": "UniProtKB:Q14242",
  "gene_symbol": "SELPLG",
  "gene_name": "P-selectin glycoprotein ligand 1"
}